vacuolar sorting signal binding [GO:0010209] (molecular function) Definition: Binding to a vacuolar sorting signal, a specific peptide sequence that acts as a signal to localize the protein within the vacuole. Sources: GOC:mah Relationships: is a type of GO:0005048 Subtypes: GO:0009940